{
  "term_label": "cytoplasm",
  "gene_symbol": "NEU4",
  "gene": "UniProtKB:Q8WWR8",
  "gene_name": "Sialidase-4",
  "term_id": "GO:0005737"
}